{
  "gene": "UniProtKB:Q8NFP9",
  "gene_symbol": "NBEA",
  "gene_name": "Neurobeachin",
  "term_label": "synapse organization",
  "term_id": "GO:0050808"
}